{
  "term_id": "GO:0005634",
  "term_label": "nucleus",
  "gene": "UniProtKB:O14503",
  "gene_symbol": "BHLHE40",
  "gene_name": "Class E basic helix-loop-helix protein 40"
}